{
  "term_label": "central nervous system development",
  "term_id": "GO:0007417",
  "gene_name": "Zinc finger protein ZIC 2",
  "gene_symbol": "ZIC2",
  "gene": "UniProtKB:O95409"
}